{
  "term_id": "GO:0005847",
  "gene_symbol": "CPSF6",
  "gene_name": "Cleavage and polyadenylation specificity factor subunit 6",
  "gene": "UniProtKB:Q16630",
  "term_label": "mRNA cleavage and polyadenylation specificity factor complex"
}